{
  "term_label": "morphogenesis of an epithelium",
  "gene_name": "Keratin, type I cuticular Ha3-I",
  "gene_symbol": "KRT33A",
  "term_id": "GO:0002009",
  "gene": "UniProtKB:O76009"
}